sinoatrial valve development [GO:0003172] (BP) Relationships: is a type of heart valve development [GO:0003170] Definition: The progression of the sinoatrial valve over time, from its formation to the mature structure. Sources: GOC:mtg_heart Also known as: SA valve development